{
  "gene_name": "2',5'-phosphodiesterase 12",
  "gene_symbol": "PDE12",
  "term_id": "GO:0005739",
  "term_label": "mitochondrion",
  "gene": "UniProtKB:Q6L8Q7"
}